positive regulation of centrosome duplication [GO:0010825] (biological process) Definition: Any process that increases the frequency, rate or extent of centrosome duplication. Centrosome duplication is the replication of a centrosome, a structure comprised of a pair of centrioles and peri-centriolar material from which a microtubule spindle apparatus is organized. Relationships: is a type of regulation of centrosome duplication [GO:0010824]; is a type of positive regulation of cell cycle process [GO:0090068]; positively regulates centrosome duplication [GO:0051298] Sources: GOC:dph, GOC:tb